cytosine catabolic process [GO:0006209] (biological process) Sources: GOC:go_curators Also known as: cytosine breakdown, cytosine catabolism, cytosine degradation Definition: The chemical reactions and pathways resulting in the breakdown of cytosine, 4-amino-2-hydroxypyrimidine, a pyrimidine derivative that is one of the five main bases found in nucleic acids; it occurs widely in cytidine derivatives. Relationships: is a type of pyrimidine nucleobase catabolic process [GO:0006208]; is a type of GO:0019858